chorismate biosynthetic process [GO:0009423] (biological process) Definition: The chemical reactions and pathways resulting in the formation of the unsymmetrical ether derived from phosphoenolpyruvate and 5-phosphoshikimic acid formed as an intermediate in the biosynthesis of aromatic amino acids and many other compounds. Relationships: is a type of dicarboxylic acid biosynthetic process [GO:0043650]; is a type of GO:0046417 Also known as: chorismate anabolism, chorismate biosynthesis, chorismate formation, chorismate synthesis, shikimate pathway, shikimate anabolism, shikimate biosynthesis, shikimate biosynthetic process, shikimate synthesis Sources: GOC:sm, ISBN:0198547684